CC tRNA cytidylyltransferase activity [GO:0052927] (molecular function) Relationships: is_a cytidylyltransferase activity [GO:0070567]; is a type of GO:0140101 References: PMID:31936900, PMID:33095240 Sources: RHEA:60008 Definition: Catalysis of the reaction: a tRNA precursor + CTP = a tRNA with a 3' CC end + 2 diphosphate. Also known as: CC-adding tRNA nucleotidyltransferase activity, CTP:tRNA cytidylyltransferase activity, CTP:3'-cytidine-tRNA cytidylyltransferase activity